{
  "term_id": "UNKNOWN:0002",
  "term_label": "Unknown biological process",
  "gene_name": "Zinc finger matrin-type protein 3",
  "gene": "UniProtKB:Q9HA38",
  "gene_symbol": "ZMAT3"
}